{
  "gene": "UniProtKB:Q9NYQ6",
  "gene_symbol": "CELSR1",
  "gene_name": "Cadherin EGF LAG seven-pass G-type receptor 1",
  "term_id": "UNKNOWN:0001",
  "term_label": "Unknown molecular function"
}